positive regulation of sphingomyelin catabolic process [GO:2000755] (biological process) Relationships: is a type of GO:0034250; is a type of positive regulation of phospholipid catabolic process [GO:0060697]; is a type of GO:2000754; positively regulates sphingomyelin catabolic process [GO:0006685] Sources: GOC:BHF Definition: Any process that activates or increases the frequency, rate or extent of sphingomyelin catabolic process. Also known as: positive regulation of sphingomyelin breakdown, positive regulation of sphingomyelin catabolism, positive regulation of sphingomyelin degradation